{
  "gene_symbol": "DCAF11",
  "gene": "UniProtKB:Q8TEB1",
  "term_id": "UNKNOWN:0001",
  "term_label": "Unknown molecular function",
  "gene_name": "DDB1- and CUL4-associated factor 11"
}